{
  "term_id": "UNKNOWN:0001",
  "term_label": "Unknown molecular function",
  "gene": "UniProtKB:Q6UWE0",
  "gene_symbol": "LRSAM1",
  "gene_name": "E3 ubiquitin-protein ligase LRSAM1"
}